{
  "term_id": "GO:0005757",
  "term_label": "mitochondrial permeability transition pore complex",
  "gene_symbol": "SLC25A4",
  "gene_name": "ADP_ATP translocase 1",
  "gene": "UniProtKB:P12235"
}